{
  "term_label": "plasma membrane",
  "gene_name": "Heat shock 70 kDa protein 6",
  "gene_symbol": "HSPA6",
  "term_id": "GO:0005886",
  "gene": "UniProtKB:P17066"
}